regulation of larval salivary gland boundary specification [GO:0045708] (biological process) Sources: GOC:go_curators, GOC:tb Subtypes: negative regulation of larval salivary gland boundary specification [GO:0045710], positive regulation of larval salivary gland boundary specification [GO:0045712] Relationships: is a type of regulation of salivary gland boundary specification [GO:0045704]; regulates larval salivary gland boundary specification [GO:0007433] Also known as: regulation of larval salivary gland determination Definition: Any process that modulates the frequency, rate or extent of salivary gland determination in a larval organism.